{
  "gene_symbol": "TMEM258",
  "term_id": "GO:0034976",
  "gene": "UniProtKB:P61165",
  "gene_name": "Transmembrane protein 258",
  "term_label": "response to endoplasmic reticulum stress"
}